positive regulation of floral organ abscission [GO:0060861] (biological process) Sources: GOC:dph, GOC:sdb_2009, GOC:tb Relationships: is a type of GO:0051094; is a type of regulation of floral organ abscission [GO:0060860]; is a type of positive regulation of reproductive process [GO:2000243]; positively regulates GO:0010227 Definition: Any process that increases the rate, frequency, or extent of floral organ shedding, the controlled shedding of floral organs.